{
  "term_id": "GO:0019372",
  "gene_symbol": "ALOX15",
  "term_label": "lipoxygenase pathway",
  "gene": "UniProtKB:P16050",
  "gene_name": "Polyunsaturated fatty acid lipoxygenase ALOX15"
}